DIF dechlorinase activity [GO:0099085] (molecular function) References: PMID:1521542, PMID:22035794 Definition: Catalysis of the reaction: 1-[(3,5-dichloro-2,6-dihydroxy-4-methoxy)phenyl]hexan-1-one = 1-[(3-chloro-2,6-dihydroxy-4-methoxy)phenyl]hexan-1-one + Cl-. Relationships: is_a GO:0016848 Also known as: 1-(3,5-dichloro-2,6-dihydroxy-4-methoxyphenyl)hexan-1-one 3(5)-dechlorinase activity, 1-[(3,5-dichloro-2,6-dihydroxy-4-methoxy)phenyl]hexan-1-one 3(5)-dechlorinase activity, DIF-1 3(5)-dechlorinase activity, DIF-1 dechlorinase activity, differentiation-inducing factor 1 dechlorinase activity, differentiation-inducing factor dechlorinase activity